leukocyte migration involved in inflammatory response [GO:0002523] (biological process) Relationships: is a type of leukocyte migration [GO:0050900]; is part of inflammatory response [GO:0006954] Also known as: immune cell migration during inflammatory response, immune cell trafficking during inflammatory response, leucocyte migration during inflammatory response, leucocyte trafficking during inflammatory response, leukocyte migration during inflammatory response, leukocyte trafficking during inflammatory response Definition: The movement of a leukocyte within or between different tissues and organs of the body contributing to an inflammatory response. Subtypes: leukocyte chemotaxis involved in inflammatory response [GO:0002232] References: PMID:14680625, PMID:14708592, PMID:7507411, PMID:8600538 Sources: GOC:add, ISBN:0781735149